apoptotic cell clearance [GO:0043277] (biological process) Also known as: apoptotic cell removal, efferocytosis, programmed cell clearance Subtypes: neutrophil clearance [GO:0097350] Note: Note that unlike mammals or Drosophila, C. elegans (and many lower organisms) do not have professional macrophages/phagocytes, instead cell corpses are engulfed by neighboring cells. Cell types that can function as engulfing cells include hypodermal cells, gonadal sheath cells, pharyngeal muscle cells, and intestinal cells. Definition: The recognition and removal of an apoptotic cell by a neighboring cell or by a phagocyte. References: PMID:14685684 Sources: GOC:rk Regulation: regulated by regulation of apoptotic cell clearance [GO:2000425]; RO_0002212 by negative regulation of apoptotic cell clearance [GO:2000426]; positively regulated by positive regulation of apoptotic cell clearance [GO:2000427] Relationships: is a type of phagocytosis [GO:0006909]